negative regulation of exocytosis [GO:0045920] (biological process) Subtypes: negative regulation of exocyst assembly [GO:0001929], negative regulation of regulated secretory pathway [GO:1903306], negative regulation of constitutive secretory pathway [GO:1903434], negative regulation of exosomal secretion [GO:1903542] Sources: GOC:go_curators Definition: Any process that stops, prevents, or reduces the frequency, rate or extent of exocytosis. Also known as: down regulation of exocytosis, down-regulation of exocytosis, downregulation of exocytosis, inhibition of exocytosis Relationships: is a type of regulation of exocytosis [GO:0017157]; is a type of negative regulation of secretion by cell [GO:1903531]; negatively regulates GO:0006887